UDP-N-acetylglucosamine-lysosomal-enzyme N-acetylglucosaminephosphotransferase activity [GO:0003976] (molecular function) Sources: EC:2.7.8.17 Definition: Catalysis of the reaction: UDP-N-acetyl-D-glucosamine + lysosomal-enzyme D-mannose = UMP + lysosomal-enzyme N-acetyl-D-glucosaminyl-phospho-D-mannose. Also known as: N-acetylglucosaminyl phosphotransferase activity, N-acetylglucosaminylphosphotransferase activity, UDP-GlcNAc:glycoprotein N-acetylglucosamine-1-phosphotransferase activity, UDP-N-acetyl-D-glucosamine:lysosomal-enzyme N-acetylglucosaminephosphotransferase activity, UDP-N-acetylglucosamine:glycoprotein N-acetylglucosamine-1-phosphotransferase activity, UDP-N-acetylglucosamine:glycoprotein N-acetylglucosaminyl-1-phosphotransferase activity, UDP-N-acetylglucosamine:lysosomal enzyme N-acetylglucosamine-1-phosphotransferase activity, lysosomal enzyme precursor acetylglucosamine-1-phosphotransferase activity Relationships: is a type of phosphotransferase activity, for other substituted phosphate groups [GO:0016780]